{
  "gene_name": "Probable G-protein coupled receptor 33",
  "gene": "UniProtKB:Q49SQ1",
  "term_label": "complement receptor activity",
  "gene_symbol": "GPR33",
  "term_id": "GO:0004875"
}